{
  "term_label": "Unknown molecular function",
  "term_id": "UNKNOWN:0001",
  "gene_symbol": "CCDC110",
  "gene": "UniProtKB:Q8TBZ0",
  "gene_name": "Coiled-coil domain-containing protein 110"
}